cellular response to cobalamin [GO:0071297] (biological process) Relationships: is a type of response to cobalamin [GO:0033590]; is a type of GO:0071295; is a type of cellular response to nitrogen compound [GO:1901699]; is a type of cellular response to oxygen-containing compound [GO:1901701] Sources: GOC:mah Definition: Any process that results in a change in state or activity of a cell (in terms of movement, secretion, enzyme production, gene expression, etc.) as a result of a cobalamin (vitamin B12) stimulus. Also known as: cellular response to vitamin B12